{
  "gene_symbol": "FAM170A",
  "gene": "UniProtKB:A1A519",
  "term_label": "nucleus",
  "gene_name": "Protein FAM170A",
  "term_id": "GO:0005634"
}